{
  "term_label": "Unknown molecular function",
  "term_id": "UNKNOWN:0001",
  "gene_name": "Uncharacterized protein C16orf46",
  "gene_symbol": "C16orf46",
  "gene": "UniProtKB:Q6P387"
}